specification of segmental identity, trunk [GO:0035292] (biological process) Definition: The specification of the characteristic structures of trunk segments, following establishment of segment boundaries. In Drosophila, the trunk segments include thoracic segments and abdominal segments A1 to A8. Identity is considered to be the aggregate of characteristics by which a structure is recognized. References: PMID:1360402 Relationships: is a type of segment specification [GO:0007379]; is part of trunk segmentation [GO:0035290] Subtypes: specification of segmental identity, thorax [GO:0007384], specification of segmental identity, abdomen [GO:0007385]